{
  "gene": "UniProtKB:Q6S8J3",
  "term_id": "GO:0005737",
  "term_label": "cytoplasm",
  "gene_name": "POTE ankyrin domain family member E",
  "gene_symbol": "POTEE"
}